{
  "term_id": "GO:0005615",
  "term_label": "extracellular space",
  "gene_symbol": "WNT5B",
  "gene_name": "Protein Wnt-5b",
  "gene": "UniProtKB:Q9H1J7"
}